LIM domain binding [GO:0030274] (molecular function) Definition: Binding to a LIM domain (for Lin-11 Isl-1 Mec-3) of a protein, a domain with seven conserved cysteine residues and a histidine, that binds two zinc ions and acts as an interface for protein-protein interactions. Relationships: is a type of protein domain specific binding [GO:0019904] Sources: GOC:go_curators, Pfam:PF00412